cellular response to topoisomerase inhibitor [GO:0072759] (biological process) Sources: GOC:mah Definition: Any process that results in a change in state or activity of a (in terms of movement, secretion, enzyme production, gene expression, etc.) as a result of a topoisomerase inhibitor stimulus. Relationships: is a type of cellular response to chemical stimulus [GO:0070887]; is a type of response to topoisomerase inhibitor [GO:0072758]